metaphase/anaphase transition of meiosis II [GO:1990950] (biological process) Relationships: is a type of metaphase/anaphase transition of meiotic cell cycle [GO:0044785]; is_a meiosis II cell cycle process [GO:0061983] Regulation: RO_0002211 by regulation of metaphase/anaphase transition of meiosis II [GO:1905189]; negatively regulated by negative regulation of metaphase/anaphase transition of meiosis II [GO:1905190]; positively regulated by positive regulation of metaphase/anaphase transition of meiosis II [GO:1905191] Definition: The cell cycle process in which a cell progresses from metaphase to anaphase as part of meiosis II. Also known as: meiosis II metaphase/anaphase transition, second meiotic metaphase/anaphase transition Sources: ISBN:0815316194